cyanoalanine nitrilase activity [GO:0047427] (molecular function) Relationships: is_a nitrilase activity [GO:0000257] Definition: Catalysis of the reaction: 3-cyano-L-alanine + 2 H2O + H+ = L-aspartate + NH4. Also known as: 3-cyano-L-alanine aminohydrolase activity, beta-cyanoalanine nitrilase activity Sources: RHEA:11188